{
  "gene_symbol": "ZC3H3",
  "term_label": "nucleus",
  "gene_name": "Zinc finger CCCH domain-containing protein 3",
  "term_id": "GO:0005634",
  "gene": "UniProtKB:Q8IXZ2"
}